{
  "term_id": "UNKNOWN:0002",
  "gene_symbol": "MATN3",
  "gene_name": "Matrilin-3",
  "gene": "UniProtKB:O15232",
  "term_label": "Unknown biological process"
}